tryptamine 4-monooxygenase activity [GO:0140382] (molecular function) References: PMID:28763571 Definition: Catalysis of the reaction: tryptamine + reduced acceptor + O2 = 4-hydroxytryptamine + acceptor + H2O. Relationships: is a type of monooxygenase activity [GO:0004497]